{
  "term_label": "volume-sensitive chloride channel activity",
  "term_id": "GO:0072320",
  "gene_symbol": "TTYH2",
  "gene": "UniProtKB:Q9BSA4",
  "gene_name": "Protein tweety homolog 2"
}